interleukin-5 receptor binding [GO:0005137] (molecular function) Definition: Binding to an interleukin-5 receptor. Relationships: is a type of cytokine receptor binding [GO:0005126]; is a type of GO:0070851 Sources: GOC:ai Also known as: IL-5, interleukin-5 receptor ligand